glycosaminoglycan metabolic process [GO:0030203] (biological process) Definition: The chemical reactions and pathways involving glycosaminoglycans, any of a group of linear polysaccharides composed of repeating disaccharide units. Also known as: glycosaminoglycan metabolism Subtypes: peptidoglycan metabolic process [GO:0000270], glycosaminoglycan biosynthetic process [GO:0006024], glycosaminoglycan catabolic process [GO:0006027], hyaluronan metabolic process [GO:0030212] Relationships: is a type of aminoglycan metabolic process [GO:0006022] References: PMID:38500384